{
  "gene_name": "DNA mismatch repair protein Msh2",
  "gene": "UniProtKB:P43246",
  "term_label": "Unknown molecular function",
  "term_id": "UNKNOWN:0001",
  "gene_symbol": "MSH2"
}